{
  "term_label": "peptide metabolic process",
  "gene_symbol": "CPE",
  "gene_name": "Carboxypeptidase E",
  "term_id": "GO:0006518",
  "gene": "UniProtKB:P16870"
}